{
  "term_label": "G protein-coupled receptor signaling pathway",
  "gene": "UniProtKB:Q8NGF7",
  "gene_name": "Olfactory receptor 5B17",
  "term_id": "GO:0007186",
  "gene_symbol": "OR5B17"
}